negative regulation of sodium ion transmembrane transport [GO:1902306] (BP) Relationships: is a type of GO:0010766; is a type of regulation of sodium ion transmembrane transport [GO:1902305]; is a type of negative regulation of cation transmembrane transport [GO:1904063]; negatively regulates sodium ion transmembrane transport [GO:0035725] References: PMID:18591664 Sources: GOC:BHF, GOC:TermGenie, GOC:mtg_cardiac_conduct_nov11, GOC:rl Subtypes: negative regulation of sodium ion export across plasma membrane [GO:1903277], GO:1903783 Also known as: down regulation of sodium ion membrane transport, down regulation of sodium ion transmembrane transport, down-regulation of sodium ion membrane transport, down-regulation of sodium ion transmembrane transport, downregulation of sodium ion membrane transport, downregulation of sodium ion transmembrane transport, negative regulation of sodium ion membrane transport, inhibition of sodium ion membrane transport, inhibition of sodium ion transmembrane transport Definition: Any process that stops, prevents or reduces the frequency, rate or extent of sodium ion transmembrane transport.